{
  "gene": "UniProtKB:Q96JY0",
  "term_id": "GO:0043565",
  "gene_symbol": "MAEL",
  "term_label": "sequence-specific DNA binding",
  "gene_name": "Protein maelstrom homolog"
}